{
  "gene_name": "Inner centromere protein",
  "gene_symbol": "INCENP",
  "gene": "UniProtKB:Q9NQS7",
  "term_id": "GO:0032133",
  "term_label": "chromosome passenger complex"
}